{
  "term_label": "microtubule cytoskeleton",
  "gene_symbol": "SEPTIN8",
  "gene": "UniProtKB:Q92599",
  "gene_name": "Septin-8",
  "term_id": "GO:0015630"
}